hepoxilin biosynthetic process [GO:0051122] (biological process) Relationships: is a type of long-chain fatty acid biosynthetic process [GO:0042759] Also known as: hepoxilin anabolism, hepoxilin biosynthesis, hepoxilin formation, hepoxilin synthesis Sources: GOC:ai Definition: The chemical reactions and pathways resulting in the formation of hepoxilins, a class of bioactive icosanoids with roles in the regulation of cell physiology.